{
  "term_label": "mitotic cell cycle",
  "term_id": "GO:0000278",
  "gene": "UniProtKB:Q8TF76",
  "gene_symbol": "HASPIN",
  "gene_name": "Serine_threonine-protein kinase haspin"
}